zeaxanthin 2-beta-hydroxylase activity [GO:0102464] (molecular function) Definition: Catalysis of the reaction: zeaxanthin + O2 + NADH + H+ = caloxanthin + H2O + NAD. References: PMID:22509387 Sources: GOC:pz Relationships: is_a GO:0016709